{
  "gene": "UniProtKB:Q6IPW1",
  "gene_name": "Uncharacterized protein C11orf71",
  "term_label": "Unknown biological process",
  "term_id": "UNKNOWN:0002",
  "gene_symbol": "C11orf71"
}